{
  "gene_name": "Peripherin-2",
  "gene_symbol": "PRPH2",
  "term_label": "Unknown molecular function",
  "gene": "UniProtKB:P23942",
  "term_id": "UNKNOWN:0001"
}